{
  "term_id": "GO:0030198",
  "gene_symbol": "MMP26",
  "gene": "UniProtKB:Q9NRE1",
  "term_label": "extracellular matrix organization",
  "gene_name": "Matrix metalloproteinase-26"
}